{
  "gene_name": "F-box and WD repeat domain containing protein 10B",
  "gene": "UniProtKB:O95170",
  "term_label": "Unknown cellular component",
  "gene_symbol": "FBXW10B",
  "term_id": "UNKNOWN:0003"
}